{
  "term_label": "olfactory receptor activity",
  "gene_symbol": "OR2L8",
  "gene": "UniProtKB:Q8NGY9",
  "gene_name": "Olfactory receptor 2L8",
  "term_id": "GO:0004984"
}